{
  "gene_symbol": "ERI1",
  "term_id": "GO:0060906",
  "gene": "UniProtKB:Q8IV48",
  "term_label": "negative regulation of regulatory ncRNA-mediated heterochromatin formation",
  "gene_name": "3'-5' exoribonuclease 1"
}